{
  "gene_name": "Immunoglobulin kappa variable 1D-13",
  "gene": "UniProtKB:A0A0B4J2D9",
  "gene_symbol": "IGKV1D-13",
  "term_id": "UNKNOWN:0001",
  "term_label": "Unknown molecular function"
}